{
  "term_label": "Unknown biological process",
  "term_id": "UNKNOWN:0002",
  "gene_name": "T cell receptor alpha joining 50 (Fragment)",
  "gene": "UniProtKB:A0A075B6X7",
  "gene_symbol": "TRAJ50"
}